D-ribulokinase activity [GO:0019150] (molecular function) Sources: EC:2.7.1.47 Relationships: is a type of phosphotransferase activity, alcohol group as acceptor [GO:0016773]; is a type of GO:0019200 Also known as: ATP:D-ribulose 5-phosphotransferase activity, D-ribulokinase (phosphorylating) Definition: Catalysis of the reaction: ATP + D-ribulose = ADP + D-ribulose 5-phosphate.